aerobic sulfur oxidation [GO:0070220] (biological process) Definition: A sulfur oxidation process that proceeds via the reaction catalyzed by sulfur dioxygenase, and requires the presence of oxygen. Sources: MetaCyc:SULFUROX-PWY Relationships: is_a GO:0019417 Also known as: aerobic sulphur oxidation